{
  "gene": "UniProtKB:P28072",
  "term_label": "cytosol",
  "gene_name": "Proteasome subunit beta type-6",
  "gene_symbol": "PSMB6",
  "term_id": "GO:0005829"
}